{
  "gene": "UniProtKB:P31997",
  "term_label": "heterophilic cell-cell adhesion",
  "gene_symbol": "CEACAM8",
  "term_id": "GO:0007157",
  "gene_name": "Carcinoembryonic antigen-related cell adhesion molecule 8"
}